{
  "gene_symbol": "VN1R4",
  "term_label": "plasma membrane",
  "gene_name": "Vomeronasal type-1 receptor 4",
  "term_id": "GO:0005886",
  "gene": "UniProtKB:Q7Z5H5"
}